{
  "gene_name": "Chromodomain-helicase-DNA-binding protein 4",
  "gene_symbol": "CHD4",
  "term_id": "GO:0042393",
  "term_label": "histone binding",
  "gene": "UniProtKB:Q14839"
}